{
  "gene_symbol": "PET117",
  "gene_name": "Protein PET117 homolog, mitochondrial",
  "term_id": "GO:0033617",
  "gene": "UniProtKB:Q6UWS5",
  "term_label": "mitochondrial respiratory chain complex IV assembly"
}